{
  "term_id": "GO:0005829",
  "term_label": "cytosol",
  "gene_name": "Phosphoglycerate mutase 2",
  "gene_symbol": "PGAM2",
  "gene": "UniProtKB:P15259"
}